retinal pigment epithelium development [GO:0003406] (biological process) Definition: The progression of the retinal pigment epithelium over time, from its initial formation to the mature structure. The retinal pigment epithelium is the melanin-containing layer of cells between the retina and the choroid that absorbs scattered and reflected light and removes waste products produced by the photoreceptor cells. Sources: GOC:ascb_2009, GOC:dph, GOC:tb Also known as: RPE development Relationships: is a type of epithelium development [GO:0060429]; is part of retina development in camera-type eye [GO:0060041]